{
  "term_label": "single-stranded DNA binding",
  "term_id": "GO:0003697",
  "gene": "UniProtKB:P36776",
  "gene_name": "Lon protease homolog, mitochondrial",
  "gene_symbol": "LONP1"
}